{
  "term_label": "dendrite membrane",
  "gene": "UniProtKB:P78334",
  "gene_name": "Gamma-aminobutyric acid receptor subunit epsilon",
  "term_id": "GO:0032590",
  "gene_symbol": "GABRE"
}